{
  "gene": "UniProtKB:P26583",
  "term_id": "GO:0006338",
  "gene_symbol": "HMGB2",
  "gene_name": "High mobility group protein B2",
  "term_label": "chromatin remodeling"
}